spindle assembly involved in female meiosis [GO:0007056] (biological process) Also known as: female meiotic spindle assembly Sources: GOC:mah Definition: The aggregation, arrangement and bonding together of a set of components to form the spindle during a meiotic cell cycle in females. An example of this is found in Drosophila melanogaster. Relationships: is a type of meiotic spindle assembly [GO:0090306]; is part of female meiotic nuclear division [GO:0007143] Subtypes: spindle assembly involved in female meiosis I [GO:0007057], spindle assembly involved in female meiosis II [GO:0007058]